{
  "term_label": "plasma membrane",
  "gene_symbol": "EPS15L1",
  "gene": "UniProtKB:Q9UBC2",
  "term_id": "GO:0005886",
  "gene_name": "Epidermal growth factor receptor substrate 15-like 1"
}